negative regulation of mitotic DNA damage checkpoint [GO:1904290] (biological process) Definition: Any process that stops, prevents or reduces the frequency, rate or extent of mitotic DNA damage checkpoint. Relationships: is a type of negative regulation of cell cycle process [GO:0010948]; is_a positive regulation of mitotic cell cycle [GO:0045931]; is a type of GO:1904289; is a type of negative regulation of DNA damage checkpoint [GO:2000002]; negatively regulates mitotic DNA damage checkpoint signaling [GO:0044773] Also known as: down regulation of mitotic DNA damage checkpoint, down-regulation of mitotic DNA damage checkpoint, downregulation of mitotic DNA damage checkpoint, inhibition of mitotic DNA damage checkpoint References: PMID:16549501 Sources: GOC:TermGenie, GOC:kmv, GO_REF:0000058